{
  "gene_symbol": "SLC16A10",
  "gene_name": "Monocarboxylate transporter 10",
  "gene": "UniProtKB:Q8TF71",
  "term_label": "thyroid hormone transport",
  "term_id": "GO:0070327"
}